{
  "gene_symbol": "LIPN",
  "term_id": "GO:0006629",
  "gene": "UniProtKB:Q5VXI9",
  "term_label": "lipid metabolic process",
  "gene_name": "Lipase member N"
}